{
  "gene_symbol": "CALB1",
  "gene": "UniProtKB:P05937",
  "gene_name": "Calbindin",
  "term_label": "nucleus",
  "term_id": "GO:0005634"
}